phenyllactate dehydrogenase (NAD+) activity [GO:0097256] (molecular function) References: PMID:10849007 Sources: GOC:pde, RHEA:38351 Relationships: is a type of GO:0140175 Note: This enzymatic activity is usually negligible, but may become prominent when phenylalanine levels are abnormally high as in the human disease phenylketonuria (PKU). Definition: Catalysis of the reaction: (R)-3-phenyllactate + NAD+ = 3-phenylpyruvate + H+ + NADH.